{
  "term_id": "GO:0005886",
  "gene": "UniProtKB:P32856",
  "term_label": "plasma membrane",
  "gene_name": "Syntaxin-2",
  "gene_symbol": "STX2"
}